{
  "gene": "UniProtKB:Q6DHV7",
  "gene_symbol": "MAPDA",
  "term_id": "GO:0006154",
  "gene_name": "Adenosine deaminase-like protein",
  "term_label": "adenosine catabolic process"
}